{
  "term_label": "protein targeting to membrane",
  "gene_symbol": "ZDHHC22",
  "term_id": "GO:0006612",
  "gene": "UniProtKB:Q8N966",
  "gene_name": "Palmitoyltransferase ZDHHC22"
}